{
  "gene": "UniProtKB:O94829",
  "gene_symbol": "IPO13",
  "term_id": "UNKNOWN:0001",
  "term_label": "Unknown molecular function",
  "gene_name": "Importin-13"
}